neutral L-amino acid transmembrane transporter activity [GO:0015175] (MF) Definition: Enables the transfer of neutral L-amino acids from one side of a membrane to the other. Neutral amino acids have side chains with no charge at pH 7.3. Sources: GOC:ai, GOC:mtg_transport, ISBN:0815340729 Also known as: neutral amino acid transporter activity, neutral amino acid transmembrane transporter activity Relationships: is_a amino acid transmembrane transporter activity [GO:0015171]; is part of GO:0015804 Subtypes: GO:0000514, beta-alanine transmembrane transporter activity [GO:0001761], neutral L-amino acid secondary active transmembrane transporter activity [GO:0005294], neutral L-amino acid:sodium symporter activity [GO:0005295], L-valine transmembrane transporter activity [GO:0005304], GO:0015182, L-glutamine transmembrane transporter activity [GO:0015186], glycine transmembrane transporter activity [GO:0015187], L-isoleucine transmembrane transporter activity [GO:0015188], GO:0015190, GO:0015193, GO:0015195, alanine transmembrane transporter activity [GO:0022858], cysteine transmembrane transporter activity [GO:0033229], homoserine transmembrane transporter activity [GO:0042970], neutral L-amino acid:sodium:chloride symporter activity [GO:0140931], broad specificity neutral L-amino acid:basic L-amino acid antiporter activity [GO:0180009]